{
  "gene_name": "Sestrin-2",
  "gene_symbol": "SESN2",
  "gene": "UniProtKB:P58004",
  "term_label": "cellular response to L-leucine",
  "term_id": "GO:0071233"
}